{
  "gene_symbol": "APOA4",
  "term_id": "GO:0055090",
  "gene": "UniProtKB:P06727",
  "term_label": "acylglycerol homeostasis",
  "gene_name": "Apolipoprotein A-IV"
}